ribonuclease P activity [GO:0004526] (molecular function) Relationships: is a type of GO:0004549; is a type of RNA endonuclease activity producing 5'-phosphomonoesters, hydrolytic mechanism [GO:0016891] Sources: EC:3.1.26.5 Also known as: RNase P, tRNA 5' leader endonuclease activity Definition: Catalysis of the endonucleolytic cleavage of RNA, removing 5' extra nucleotides from tRNA precursor.